{
  "gene": "UniProtKB:O00478",
  "term_label": "regulation of cytokine production",
  "gene_symbol": "BTN3A3",
  "term_id": "GO:0001817",
  "gene_name": "Butyrophilin subfamily 3 member A3"
}